lignan catabolic process [GO:0046273] (biological process) Definition: The chemical reactions and pathways resulting in the breakdown of lignans, any member of a class of plant metabolites related to lignins. Lignans are usually found as phenylpropanoid dimers in which the phenylpropanoid units are linked tail to tail and thus having a 2,3 dibenzylbutane skeleton, but higher oligomers can also exist. Relationships: is a type of GO:0009806; is_a phenylpropanoid catabolic process [GO:0046271] References: PMID:10074466 Sources: GOC:jl Subtypes: (-)-pinoresinol catabolic process [GO:1902123], (+)-pinoresinol catabolic process [GO:1902125], (-)-lariciresinol catabolic process [GO:1902128], GO:1902131, GO:1902134, (-)-secoisolariciresinol catabolic process [GO:1902137] Also known as: lignan breakdown, lignan catabolism, lignan degradation